{
  "term_id": "GO:0005886",
  "gene_name": "Membrane progestin receptor alpha",
  "term_label": "plasma membrane",
  "gene_symbol": "PAQR7",
  "gene": "UniProtKB:Q86WK9"
}